{
  "term_id": "GO:0005891",
  "gene": "UniProtKB:Q02641",
  "term_label": "voltage-gated calcium channel complex",
  "gene_name": "Voltage-dependent L-type calcium channel subunit beta-1",
  "gene_symbol": "CACNB1"
}